{
  "term_label": "Unknown biological process",
  "gene_name": "Tuftelin",
  "term_id": "UNKNOWN:0002",
  "gene": "UniProtKB:Q9NNX1",
  "gene_symbol": "TUFT1"
}